connecting tubule development [GO:0072027] (biological process) Sources: GOC:mtg_kidney_jan10 Also known as: connecting duct development Subtypes: GO:0061272, GO:0072286 Relationships: is a type of GO:0072080 Definition: The process whose specific outcome is the progression of the connecting tubule over time, from its formation to the mature structure. The connecting tubule is a tubular segment of the nephron; it connects the distal convoluted tubule to the collecting duct.